{
  "gene": "UniProtKB:O43194",
  "gene_symbol": "GPR39",
  "gene_name": "G-protein coupled receptor 39",
  "term_label": "Unknown cellular component",
  "term_id": "UNKNOWN:0003"
}